{
  "term_id": "GO:0070971",
  "gene_symbol": "SAR1B",
  "gene": "UniProtKB:Q9Y6B6",
  "term_label": "endoplasmic reticulum exit site",
  "gene_name": "GTP-binding protein SAR1b"
}